{
  "term_label": "Unknown cellular component",
  "gene_symbol": "TRAV1-1",
  "gene": "UniProtKB:A0A0B4J248",
  "gene_name": "T cell receptor alpha variable 1-1",
  "term_id": "UNKNOWN:0003"
}